positive regulation of vesicle fusion [GO:0031340] (biological process) Subtypes: positive regulation of synaptic vesicle fusion to presynaptic active zone membrane [GO:0031632], positive regulation of SNARE complex assembly [GO:0035543], positive regulation of Golgi vesicle fusion to target membrane [GO:0048215], positive regulation of vesicle fusion with Golgi apparatus [GO:0106216], positive regulation of autophagosome-lysosome fusion [GO:0160177], positive regulation of endosomal vesicle fusion [GO:1905363] Also known as: up regulation of vesicle fusion, up-regulation of vesicle fusion, upregulation of vesicle fusion, activation of vesicle fusion, stimulation of vesicle fusion Definition: Any process that activates or increases the frequency, rate or extent of vesicle fusion. Relationships: is_a GO:0010638; is a type of regulation of vesicle fusion [GO:0031338]; is a type of positive regulation of transport [GO:0051050]; RO_0002213 vesicle fusion [GO:0006906] Sources: GOC:mah